negative regulation of telomeric D-loop disassembly [GO:1905839] (biological process) References: PMID:15200954 Sources: GOC:BHF, GOC:BHF_telomere, GOC:TermGenie, GOC:nc, GO_REF:0000058 Relationships: is_a GO:1904534; is_a GO:1905838; negatively regulates telomeric D-loop disassembly [GO:0061820] Definition: Any process that stops, prevents or reduces the frequency, rate or extent of telomeric D-loop disassembly. Also known as: down regulation of telomeric D-loop disassembly, down-regulation of telomeric D-loop disassembly, downregulation of telomeric D-loop disassembly, inhibition of telomeric D-loop disassembly